{
  "term_id": "GO:0005882",
  "gene_symbol": "SYNM",
  "term_label": "intermediate filament",
  "gene_name": "Synemin",
  "gene": "UniProtKB:O15061"
}